establishment of protein localization [GO:0045184] (biological process) Definition: The directed movement of a protein to a specific location. Sources: GOC:bf Also known as: establishment of protein localisation, protein positioning, protein recruitment Relationships: is a type of establishment of localization [GO:0051234] Subtypes: GO:0006605, protein transport [GO:0015031], establishment of protein localization to extracellular region [GO:0035592], establishment of protein localization to juxtaparanode region of axon [GO:0071206], establishment of protein localization to organelle [GO:0072594], establishment of protein localization to membrane [GO:0090150] Regulation: regulated by GO:0070201; negatively regulated by negative regulation of establishment of protein localization [GO:1904950]; RO_0002213 by positive regulation of establishment of protein localization [GO:1904951]